{
  "gene_symbol": "HSPB1",
  "term_id": "GO:0051082",
  "gene_name": "Heat shock protein beta-1",
  "term_label": "unfolded protein binding",
  "gene": "UniProtKB:P04792"
}